1-phosphatidylinositol-4-phosphate 3-kinase activity [GO:0035005] (molecular function) Sources: EC:2.7.1.154, RHEA:18373 Relationships: is a type of phosphatidylinositol kinase activity [GO:0052742] Also known as: phosphatidylinositol-4-phosphate 3-kinase activity, C2-domain-containing phosphoinositide 3-kinase activity, phosphatidylinositol 3-kinase activity, class I, phosphatidylinositol 3-kinase activity, class II, phosphatidylinositol 3-kinase, class I, catalyst activity, ATP:1-phosphatidyl-1D-myo-inositol-4-phosphate 3-phosphotransferase activity, type II phosphoinositide 3-kinase activity Definition: Catalysis of the reaction: a 1-phosphatidyl-1D-myo-inositol 4-phosphate + ATP = a 1-phosphatidyl-1D-myo-inositol 3,4-bisphosphate + ADP + H+.